{
  "gene_symbol": "FBXL18",
  "term_id": "UNKNOWN:0003",
  "gene_name": "F-box_LRR-repeat protein 18",
  "term_label": "Unknown cellular component",
  "gene": "UniProtKB:Q96ME1"
}